maintenance of protein location in vacuole [GO:0072667] (biological process) Relationships: is a type of maintenance of protein localization in organelle [GO:0072595]; is part of protein localization to vacuole [GO:0072665]; occurs in vacuole [GO:0005773] Definition: Any process in which a protein is maintained in a specific location in a vacuole, and is prevented from moving elsewhere. Sources: GOC:mah